{
  "gene_symbol": "AP3D1",
  "term_id": "GO:0043195",
  "gene_name": "AP-3 complex subunit delta-1",
  "term_label": "terminal bouton",
  "gene": "UniProtKB:O14617"
}